{
  "gene_name": "Pre-mRNA-processing-splicing factor 8",
  "term_id": "GO:0071013",
  "gene_symbol": "PRPF8",
  "term_label": "catalytic step 2 spliceosome",
  "gene": "UniProtKB:Q6P2Q9"
}